{
  "term_label": "plasma membrane",
  "gene": "UniProtKB:Q8NGH3",
  "gene_symbol": "OR2D3",
  "term_id": "GO:0005886",
  "gene_name": "Olfactory receptor 2D3"
}